formylaspartate deformylase activity [GO:0047902] (molecular function) Definition: Catalysis of the reaction: N-formyl-L-aspartate + H2O = formate + L-aspartate. Relationships: is a type of hydrolase activity, acting on carbon-nitrogen (but not peptide) bonds, in linear amides [GO:0016811] Sources: EC:3.5.1.8, MetaCyc:FORMYLASPARTATE-DEFORMYLASE-RXN Also known as: N-formyl-L-aspartate amidohydrolase activity, formylaspartic formylase (formylase I, formylase II)